{
  "gene": "UniProtKB:Q96BF3",
  "gene_name": "Transmembrane and immunoglobulin domain-containing protein 2",
  "gene_symbol": "TMIGD2",
  "term_label": "Unknown molecular function",
  "term_id": "UNKNOWN:0001"
}